{
  "gene": "UniProtKB:A6NM62",
  "gene_name": "Leucine-rich repeat-containing protein 53",
  "gene_symbol": "LRRC53",
  "term_label": "Unknown biological process",
  "term_id": "UNKNOWN:0002"
}